{
  "term_label": "Unknown biological process",
  "gene_name": "Kita-kyushu lung cancer antigen 1",
  "term_id": "UNKNOWN:0002",
  "gene": "UniProtKB:Q5H943",
  "gene_symbol": "CT83"
}